{
  "term_label": "ribosomal subunit export from nucleus",
  "gene_symbol": "RAN",
  "gene": "UniProtKB:P62826",
  "term_id": "GO:0000054",
  "gene_name": "GTP-binding nuclear protein Ran"
}